{
  "term_id": "GO:0007219",
  "gene_symbol": "RBPJ",
  "gene_name": "Recombining binding protein suppressor of hairless",
  "term_label": "Notch signaling pathway",
  "gene": "UniProtKB:Q06330"
}